semicircular canal development [GO:0060872] (biological process) Subtypes: GO:0060873, posterior semicircular canal development [GO:0060874], lateral semicircular canal development [GO:0060875] Relationships: is a type of tube development [GO:0035295]; is part of inner ear development [GO:0048839] Definition: The progression of the semicircular canal from its initial formation to the mature structure. Sources: GOC:dph, GOC:sdb_2009, GOC:tb